malonate-semialdehyde dehydrogenase (acetylating) activity [GO:0018478] (MF) Relationships: is a type of oxidoreductase activity, acting on the aldehyde or oxo group of donors, NAD or NADP as acceptor [GO:0016620] Definition: Catalysis of the reaction: 3-oxopropanoate + CoA + NAD(P)+ = acetyl-CoA + CO2 + NAD(P)H. Sources: EC:1.2.1.18 Also known as: malonic semialdehyde oxidative decarboxylase activity, 3-oxopropanoate:NAD(P)+ oxidoreductase (decarboxylating, CoA-acetylating)